stem cell factor receptor binding [GO:0005173] (molecular function) Also known as: SCFR binding, KIT binding, SCF, stem cell factor, stem cell factor receptor ligand Definition: Binding to a stem cell factor receptor (SCFR), a type III transmembrane kinase receptor. Relationships: is a type of cytokine receptor binding [GO:0005126] References: PMID:10698217 Sources: GOC:jl